{
  "term_label": "Unknown biological process",
  "term_id": "UNKNOWN:0002",
  "gene_symbol": "IBA57-DT",
  "gene_name": "Putative uncharacterized protein IBA57-DT",
  "gene": "UniProtKB:B1ANH7"
}